{
  "gene": "UniProtKB:Q6NSX1",
  "term_label": "Unknown cellular component",
  "gene_symbol": "CCDC70",
  "gene_name": "Coiled-coil domain-containing protein 70",
  "term_id": "UNKNOWN:0003"
}